{
  "gene_symbol": "ZNF142",
  "gene_name": "Zinc finger protein 142",
  "term_id": "GO:0005634",
  "gene": "UniProtKB:P52746",
  "term_label": "nucleus"
}